{
  "gene_name": "RNA-binding motif protein, Y chromosome, family 1 member B",
  "gene": "UniProtKB:A6NDE4",
  "term_id": "GO:0005681",
  "gene_symbol": "RBMY1B",
  "term_label": "spliceosomal complex"
}